{
  "gene_name": "Serine_threonine-protein kinase PLK3",
  "term_label": "cytoplasm",
  "term_id": "GO:0005737",
  "gene": "UniProtKB:Q9H4B4",
  "gene_symbol": "PLK3"
}